transcription factor TFIIIC1 complex [GO:0034734] (cellular component) References: PMID:11433012, PMID:15096501 Sources: GOC:mah Definition: A transcription factor complex that forms part of the TFIIIC complex, observed in human. The complex is poorly characterized, but contains the 250-kDa form of HsBdp1, and is thought to include nuclear factor 1 (NF1). It stimulates binding by human TFIIIC2 and is required for transcription activity. Relationships: is a type of RNA polymerase III transcription regulator complex [GO:0090576]; is part of transcription factor TFIIIC complex [GO:0000127]